glucuronate-1-phosphate uridylyltransferase activity [GO:0047350] (molecular function) Sources: EC:2.7.7.44, RHEA:16325 Also known as: UTP:glucuronate-1-phosphate uridylyltransferase activity, UDP-D-glucuronic acid pyrophosphorylase activity, UDP-glucuronate pyrophosphorylase activity, UDP-glucuronic acid pyrophosphorylase activity, UTP:1-phospho-alpha-D-glucuronate uridylyltransferase activity, uridine diphosphoglucuronic pyrophosphorylase activity Relationships: is a type of GO:0070569 Definition: Catalysis of the reaction: 1-phospho-alpha-D-glucuronate + UTP = diphosphate + UDP-alpha-D-glucuronate.